{
  "gene_symbol": "OPN5",
  "gene": "UniProtKB:Q6U736",
  "term_id": "GO:0007186",
  "gene_name": "Opsin-5",
  "term_label": "G protein-coupled receptor signaling pathway"
}